{
  "term_id": "UNKNOWN:0001",
  "gene": "UniProtKB:Q8IZ13",
  "term_label": "Unknown molecular function",
  "gene_name": "Protein FAM200C",
  "gene_symbol": "FAM200C"
}